{
  "gene_name": "Sperm acrosome-associated protein 7",
  "term_id": "GO:0001669",
  "term_label": "acrosomal vesicle",
  "gene": "UniProtKB:Q96KW9",
  "gene_symbol": "SPACA7"
}